organophosphate ester transmembrane transporter activity [GO:0015605] (molecular function) Sources: GOC:mcc Subtypes: glycerophosphodiester transmembrane transporter activity [GO:0001406], nucleotide-sugar transmembrane transporter activity [GO:0005338], nucleotide-sulfate transmembrane transporter activity [GO:0005340], acetyl-CoA transmembrane transporter activity [GO:0008521], hexose phosphate transmembrane transporter activity [GO:0015119], glycerol-3-phosphate transmembrane transporter activity [GO:0015169], nucleotide transmembrane transporter activity [GO:0015215], coenzyme A transmembrane transporter activity [GO:0015228], GO:0015527, ABC-type fatty-acyl-CoA transporter activity [GO:0015607], pyridoxal phosphate transmembrane transporter activity [GO:0031926], glycerone phosphate:phosphate antiporter activity [GO:0051407], GO:0051978, triose-phosphate transmembrane transporter activity [GO:0071917], phosphoenolpyruvate transmembrane transporter activity [GO:0089721], GO:0090422, isopentenyl pyrophosphate transmembrane transporter activity [GO:0170045] Definition: Enables the transfer of organophosphate esters from one side of a membrane to the other. Organophosphate esters are small organic molecules containing phosphate ester bonds. Relationships: is a type of transmembrane transporter activity [GO:0022857]; is part of organophosphate ester transport [GO:0015748]